{
  "gene_name": "Immunoglobulin kappa variable 2D-30",
  "gene": "UniProtKB:A0A075B6S6",
  "term_label": "immunoglobulin complex",
  "gene_symbol": "IGKV2D-30",
  "term_id": "GO:0019814"
}